interleukin-13 receptor complex [GO:0005898] (cellular component) Also known as: IL-13 receptor complex Definition: A protein complex that binds interleukin-13; consists of two chains, interleukin-13 receptor alpha1 chain and interleukin-4 receptor alpha chain. Relationships: is a type of plasma membrane signaling receptor complex [GO:0098802] References: PMID:8552669, PMID:9013879